Bunina body [GO:0097407] (cellular component) Relationships: is a type of inclusion body [GO:0016234] References: PMID:18026741 Sources: NIF_Subcellular:nlx_subcell_20090101 Definition: Small granular inclusions (about 1-3 microns in diameter) found in the anterior horn cells, and appearing either singly or in a group. Sometimes they are arranged in small beaded chains. Bunina bodies express cystatin C and consist of electron-dense amorphous material that contains tubules or vesicular structures. The amorphous material frequently includes a cytoplasmic island containing neurofilaments and other micro-organelles.